{
  "gene_symbol": "KASH5",
  "term_label": "chromosome localization to nuclear envelope involved in homologous chromosome segregation",
  "gene_name": "Protein KASH5",
  "term_id": "GO:0090220",
  "gene": "UniProtKB:Q8N6L0"
}